{
  "gene": "UniProtKB:Q9NQ88",
  "gene_name": "Fructose-2,6-bisphosphatase TIGAR",
  "gene_symbol": "TIGAR",
  "term_label": "regulation of pentose-phosphate shunt",
  "term_id": "GO:0043456"
}